positive regulation of peptidyl-tyrosine phosphorylation [GO:0050731] (biological process) Also known as: up regulation of peptidyl-tyrosine phosphorylation, up-regulation of peptidyl-tyrosine phosphorylation, upregulation of peptidyl-tyrosine phosphorylation, activation of peptidyl-tyrosine phosphorylation, stimulation of peptidyl-tyrosine phosphorylation Relationships: is_a positive regulation of protein phosphorylation [GO:0001934]; is a type of regulation of peptidyl-tyrosine phosphorylation [GO:0050730]; positively regulates peptidyl-tyrosine phosphorylation [GO:0018108] Definition: Any process that activates or increases the frequency, rate or extent of the phosphorylation of peptidyl-tyrosine. Sources: GOC:ai Subtypes: positive regulation of tyrosine phosphorylation of STAT protein [GO:0042531], positive regulation of protein tyrosine kinase activity [GO:0061098], positive regulation of peptidyl-tyrosine autophosphorylation [GO:1900086]